{
  "term_label": "Unknown biological process",
  "term_id": "UNKNOWN:0002",
  "gene_name": "Equilibrative nucleoside transporter 3",
  "gene_symbol": "SLC29A3",
  "gene": "UniProtKB:Q9BZD2"
}